{
  "term_label": "pICln-Sm protein complex",
  "gene_symbol": "SNRPE",
  "gene_name": "Small nuclear ribonucleoprotein E",
  "gene": "UniProtKB:P62304",
  "term_id": "GO:0034715"
}